{
  "term_label": "histidine transport",
  "gene": "UniProtKB:Q8N697",
  "gene_name": "Solute carrier family 15 member 4",
  "term_id": "GO:0015817",
  "gene_symbol": "SLC15A4"
}